N-terminal protein amino acid deamination [GO:0031363] (biological process) Sources: GOC:mah Subtypes: N-terminal protein amino acid deamination, from amino carbon [GO:0018058], N-terminal protein amino acid deamination, from side chain [GO:0031364] Relationships: is_a GO:0031365 Definition: The removal of an amino group from the N-terminal amino acid residue of a protein.